nucleoplasmic side of nuclear pore [GO:1990875] (cellular component) Also known as: nucleoplasmic side of NPC, nucleoplasmic side of nuclear pore complex, nucleoplasmic side of nucleopore Definition: The side of the nuclear pore complex (NPC) that faces the nucleoplasm. Relationships: is_a GO:0110165; BFO_0000050 GO:0005643 References: PMID:8422679